xylan alpha-1,2-glucuronosidase activity [GO:0033939] (molecular function) Also known as: 1,2-alpha-glucuronidase activity, alpha-(1->2)-glucuronidase activity, xylan alpha-D-1,2-(4-O-methyl)glucuronohydrolase activity Relationships: is_a hydrolase activity, hydrolyzing O-glycosyl compounds [GO:0004553] Sources: EC:3.2.1.131 Definition: Catalysis of the hydrolysis of alpha-D-(1->2)-(4-O-methyl)glucuronosyl links in the main chain of hardwood xylans.